{
  "term_id": "GO:0003743",
  "gene_symbol": "EIF1AY",
  "gene_name": "Eukaryotic translation initiation factor 1A, Y-chromosomal",
  "gene": "UniProtKB:O14602",
  "term_label": "translation initiation factor activity"
}